{
  "term_label": "retinol transport",
  "gene": "UniProtKB:P02753",
  "term_id": "GO:0034633",
  "gene_symbol": "RBP4",
  "gene_name": "Retinol-binding protein 4"
}